{
  "term_id": "GO:0006874",
  "term_label": "intracellular calcium ion homeostasis",
  "gene_symbol": "ATP13A4",
  "gene_name": "Probable cation-transporting ATPase 13A4",
  "gene": "UniProtKB:Q4VNC1"
}